photosynthesis, dark reaction [GO:0019685] (biological process) Definition: A complex cycle of enzyme-mediated reactions which catalyzes the reduction of carbon dioxide to sugar. As well as carbon dioxide the cycle requires reducing power in the form of reduced nicotinamide adenine dinucleotide phosphate (NADP) and chemical energy in the form of adenosine triphosphate (ATP). The reduced NADP (NADPH) and ATP are produced by the 'light' reactions. Relationships: is a type of carbohydrate biosynthetic process [GO:0016051]; is part of photosynthesis [GO:0015979] Sources: ISBN:0582015952 Regulation: RO_0002211 by GO:0010110 Subtypes: C4 photosynthesis [GO:0009760], GO:0009761, reductive pentose-phosphate cycle [GO:0019253]